{
  "term_id": "UNKNOWN:0002",
  "gene": "UniProtKB:Q9H974",
  "gene_name": "Queuine tRNA-ribosyltransferase accessory subunit 2",
  "term_label": "Unknown biological process",
  "gene_symbol": "QTRT2"
}